high-mannose-oligosaccharide beta-1,4-N-acetylglucosaminyltransferase activity [GO:0033827] (molecular function) Relationships: is a type of acetylglucosaminyltransferase activity [GO:0008375] Sources: EC:2.4.1.197 Also known as: UDP-GlcNAc:oligosaccharide beta-N-acetylglucosaminyltransferase activity, UDP-N-acetyl-D-glucosamine:high-mannose-oligosaccharide beta-1,4-N-acetylglucosaminyltransferase activity, acetylglucosamine-oligosaccharide acetylglucosaminyltransferase activity, uridine diphosphoacetylglucosamine-oligosaccharide acetylglucosaminyltransferase activity Definition: Catalysis of the transfer of an N-acetyl-D-glucosamine residue from UDP-N-acetyl-D-glucosamine to the 4-position of a mannose linked alpha-1,6 to the core mannose of high-mannose oligosaccharides produced by Dictyostelium discoideum.